{
  "gene_symbol": "MARCHF7",
  "gene": "UniProtKB:Q9H992",
  "term_label": "protein autoubiquitination",
  "term_id": "GO:0051865",
  "gene_name": "E3 ubiquitin-protein ligase MARCHF7"
}